meiosis II cytokinesis [GO:0007111] (biological process) Sources: GOC:mtg_cell_cycle Relationships: is_a meiotic cytokinesis [GO:0033206]; is a type of meiosis II cell cycle process [GO:0061983] Also known as: cytokinesis after meiosis II Definition: A cell cycle process that results in the division of the cytoplasm of a cell after meiosis II, resulting in the separation of the original cell into two daughter cells.